{
  "gene_name": "DNA excision repair protein ERCC-8",
  "gene": "UniProtKB:Q13216",
  "term_id": "GO:0043161",
  "gene_symbol": "ERCC8",
  "term_label": "proteasome-mediated ubiquitin-dependent protein catabolic process"
}